{
  "term_label": "acetylcholine-gated monoatomic cation-selective channel activity",
  "gene_name": "Neuronal acetylcholine receptor subunit alpha-7",
  "gene_symbol": "CHRNA7",
  "term_id": "GO:0022848",
  "gene": "UniProtKB:P36544"
}